negative regulation of plant-type cell wall cellulose biosynthetic process [GO:2001010] (biological process) Definition: Any process that stops, prevents or reduces the frequency, rate or extent of plant-type cell wall cellulose biosynthetic process. Sources: GOC:mengo_curators Also known as: negative regulation of cell wall cellulose biosynthesis, negative regulation of cellulose biosynthesis during cell wall biosynthesis Relationships: is a type of negative regulation of cellulose biosynthetic process [GO:2001007]; is a type of GO:2001009; negatively regulates plant-type cell wall cellulose biosynthetic process [GO:0052324]